{
  "gene_name": "Protein O-mannosyl-transferase TMTC1",
  "term_label": "protein O-linked glycosylation via mannose",
  "gene": "UniProtKB:Q8IUR5",
  "gene_symbol": "TMTC1",
  "term_id": "GO:0035269"
}